positive regulation of interleukin-13 production [GO:0032736] (biological process) Sources: GOC:mah Definition: Any process that activates or increases the frequency, rate, or extent of interleukin-13 production. Also known as: positive regulation of IL-13 production, up regulation of interleukin-13 production, up-regulation of interleukin-13 production, upregulation of interleukin-13 production, activation of interleukin-13 production, positive regulation of interleukin-13 biosynthetic process, positive regulation of interleukin-13 secretion, stimulation of interleukin-13 production Relationships: is a type of GO:0001819; is a type of regulation of interleukin-13 production [GO:0032656]; positively regulates interleukin-13 production [GO:0032616]